{
  "term_id": "UNKNOWN:0003",
  "gene": "UniProtKB:A0A494C0I6",
  "gene_name": "Uncharacterized protein",
  "gene_symbol": "A0A494C0I6",
  "term_label": "Unknown cellular component"
}